{
  "gene": "UniProtKB:O15467",
  "term_label": "chemokine-mediated signaling pathway",
  "gene_name": "C-C motif chemokine 16",
  "gene_symbol": "CCL16",
  "term_id": "GO:0070098"
}